type 5 somatostatin receptor binding [GO:0031882] (molecular function) Definition: Binding to a type 5 somatostatin receptor. Sources: GOC:mah, GOC:nln Relationships: is a type of GO:0031877 Also known as: type 5 somatostatin receptor ligand